{
  "term_id": "UNKNOWN:0003",
  "gene_symbol": "SLC35F4",
  "term_label": "Unknown cellular component",
  "gene": "UniProtKB:A4IF30",
  "gene_name": "Solute carrier family 35 member F4"
}